{
  "term_id": "UNKNOWN:0001",
  "gene_symbol": "TRAPPC9",
  "term_label": "Unknown molecular function",
  "gene": "UniProtKB:Q96Q05",
  "gene_name": "Trafficking protein particle complex subunit 9"
}